positive regulation of chorionic trophoblast cell proliferation [GO:1901384] (biological process) Also known as: up regulation of chorionic trophoblast cell proliferation, up-regulation of chorionic trophoblast cell proliferation, upregulation of chorionic trophoblast cell proliferation, activation of chorionic trophoblast cell proliferation Relationships: is a type of GO:0008284; is a type of regulation of chorionic trophoblast cell proliferation [GO:1901382]; positively regulates chorionic trophoblast cell proliferation [GO:0097360] Definition: Any process that activates or increases the frequency, rate or extent of chorionic trophoblast cell proliferation. Sources: GOC:BHF, GOC:TermGenie